regulation of defense response by callose deposition [GO:2000071] (biological process) Also known as: regulation of callose deposition during defense response, regulation of callose localization during defense response Sources: GOC:obol Relationships: is a type of regulation of defense response [GO:0031347]; is a type of GO:0032879; regulates defense response by callose deposition [GO:0052542] Definition: Any process that modulates the frequency, rate or extent of defense response by callose deposition.